{
  "gene_symbol": "TRAJ29",
  "gene_name": "T cell receptor alpha joining 29 (Fragment)",
  "term_id": "UNKNOWN:0002",
  "term_label": "Unknown biological process",
  "gene": "UniProtKB:A0A075B711"
}